{
  "gene": "UniProtKB:Q9NUP9",
  "term_id": "GO:0045202",
  "term_label": "synapse",
  "gene_name": "Protein lin-7 homolog C",
  "gene_symbol": "LIN7C"
}